negative regulation of vascular endothelial growth factor production [GO:1904046] (biological process) Relationships: is a type of negative regulation of cytokine production [GO:0001818]; is a type of regulation of vascular endothelial growth factor production [GO:0010574]; negatively regulates GO:0010573 References: PMID:19404486 Sources: GOC:TermGenie, GO_REF:0000058 Also known as: down regulation of VEGF production, down regulation of vascular endothelial growth factor production, down-regulation of VEGF production, down-regulation of vascular endothelial growth factor production, downregulation of VEGF production, downregulation of vascular endothelial growth factor production, negative regulation of VEGF production, inhibition of VEGF production, inhibition of vascular endothelial growth factor production Definition: Any process that stops, prevents or reduces the frequency, rate or extent of vascular endothelial growth factor production.